{
  "term_label": "cortical actin cytoskeleton",
  "gene_symbol": "SHROOM1",
  "gene_name": "Protein Shroom1",
  "gene": "UniProtKB:Q2M3G4",
  "term_id": "GO:0030864"
}